{
  "term_label": "deacylase activity",
  "gene": "UniProtKB:Q75T13",
  "gene_name": "GPI inositol-deacylase",
  "term_id": "GO:0160215",
  "gene_symbol": "PGAP1"
}